citrate:proton symporter activity [GO:0015531] (molecular function) Also known as: citrate:hydrogen symporter activity Definition: Enables the transfer of a solute or solutes from one side of a membrane to the other according to the reaction: citrate(out) + H+(out) = citrate(in) + H+(in). Sources: TC:2.A.1.6.1 Relationships: is_a solute:proton symporter activity [GO:0015295]; is_a citrate secondary active transmembrane transporter activity [GO:0071913]